{
  "gene_symbol": "H3C13",
  "term_id": "GO:0031507",
  "term_label": "heterochromatin formation",
  "gene": "UniProtKB:Q71DI3",
  "gene_name": "Histone H3.2"
}